{
  "term_label": "plasma membrane",
  "term_id": "GO:0005886",
  "gene_name": "Cell division control protein 42 homolog",
  "gene_symbol": "CDC42",
  "gene": "UniProtKB:P60953"
}